negative regulation of optical nerve axon regeneration [GO:1905592] (biological process) Relationships: is a type of negative regulation of axon regeneration [GO:0048681]; is a type of regulation of optical nerve axon regeneration [GO:1905591]; negatively regulates optical nerve axon regeneration [GO:0101027] References: PMID:16699509 Sources: GOC:TermGenie, GO_REF:0000058 Definition: Any process that stops, prevents or reduces the frequency, rate or extent of optical nerve axon regeneration. Also known as: down regulation of optical nerve axon regeneration, down-regulation of optical nerve axon regeneration, downregulation of optical nerve axon regeneration, inhibition of optical nerve axon regeneration